{
  "term_id": "GO:1904262",
  "gene": "UniProtKB:Q8WTW4",
  "gene_name": "GATOR complex protein NPRL2",
  "term_label": "negative regulation of TORC1 signaling",
  "gene_symbol": "NPRL2"
}